{
  "gene_symbol": "C21orf140",
  "gene": "UniProtKB:B9A014",
  "term_label": "Unknown cellular component",
  "term_id": "UNKNOWN:0003",
  "gene_name": "Uncharacterized protein C21orf140"
}